{
  "gene_symbol": "CYP7B1",
  "term_id": "UNKNOWN:0003",
  "gene": "UniProtKB:O75881",
  "term_label": "Unknown cellular component",
  "gene_name": "Cytochrome P450 7B1"
}